{
  "gene_symbol": "KCNC3",
  "gene_name": "Potassium voltage-gated channel subfamily C member 3",
  "gene": "UniProtKB:Q14003",
  "term_label": "voltage-gated potassium channel complex",
  "term_id": "GO:0008076"
}